{
  "term_label": "elongator holoenzyme complex",
  "gene_symbol": "ELP4",
  "term_id": "GO:0033588",
  "gene": "UniProtKB:Q96EB1",
  "gene_name": "Elongator complex protein 4"
}